{
  "gene": "UniProtKB:Q99819",
  "gene_name": "Rho GDP-dissociation inhibitor 3",
  "term_label": "Rho GDP-dissociation inhibitor activity",
  "term_id": "GO:0005094",
  "gene_symbol": "ARHGDIG"
}